mesenchymal-endodermal cell signaling [GO:0060497] (biological process) Also known as: mesenchymal-endodermal cell signalling Sources: GOC:dph Definition: Any process that mediates the transfer of information between a mesenchymal cell and an endodermal cell. Subtypes: mesenchymal-endodermal cell signaling involved in lung induction [GO:0060493] Relationships: is a type of cell-cell signaling [GO:0007267]